{
  "gene_name": "Olfactory receptor 8B4",
  "gene_symbol": "OR8B4",
  "term_label": "sensory perception of smell",
  "term_id": "GO:0007608",
  "gene": "UniProtKB:Q96RC9"
}